dopamine neurotransmitter receptor activity [GO:0004952] (molecular function) Subtypes: dopamine neurotransmitter receptor activity, coupled via Gs [GO:0001588], dopamine neurotransmitter receptor activity, coupled via Gi/Go [GO:0001591] Relationships: is a type of postsynaptic neurotransmitter receptor activity [GO:0098960]; is part of synaptic transmission, dopaminergic [GO:0001963]; is part of GO:0007212; has part GO:0035240 Definition: Combining with the neurotransmitter dopamine to initiate a change in cell activity. References: PMID:21711983 Sources: GOC:PARL, IUPHAR_GPCR:1282